regulation of antifungal peptide secretion [GO:0002800] (biological process) Sources: GOC:add Definition: Any process that modulates the frequency, rate, or extent of antifungal peptide secretion. Subtypes: negative regulation of antifungal peptide secretion [GO:0002801], positive regulation of antifungal peptide secretion [GO:0002802] Relationships: is a type of GO:0002788; is a type of regulation of antimicrobial peptide secretion [GO:0002794]; regulates antifungal peptide secretion [GO:0002782]